{
  "gene_symbol": "AP1M1",
  "term_label": "Golgi to vacuole transport",
  "term_id": "GO:0006896",
  "gene": "UniProtKB:Q9BXS5",
  "gene_name": "AP-1 complex subunit mu-1"
}